{
  "gene_name": "Zinc finger protein 367",
  "gene_symbol": "ZNF367",
  "term_id": "GO:0005634",
  "gene": "UniProtKB:Q7RTV3",
  "term_label": "nucleus"
}